{
  "term_label": "negative regulation of apoptotic process",
  "gene": "UniProtKB:Q9P1W9",
  "gene_symbol": "PIM2",
  "gene_name": "Serine_threonine-protein kinase pim-2",
  "term_id": "GO:0043066"
}